{
  "term_label": "establishment or maintenance of cell polarity regulating cell shape",
  "gene": "UniProtKB:Q9HBI0",
  "gene_name": "Gamma-parvin",
  "gene_symbol": "PARVG",
  "term_id": "GO:0071963"
}